{
  "term_id": "UNKNOWN:0001",
  "term_label": "Unknown molecular function",
  "gene_symbol": "PI15",
  "gene": "UniProtKB:O43692",
  "gene_name": "Peptidase inhibitor 15"
}